{
  "gene": "UniProtKB:O75841",
  "term_id": "UNKNOWN:0002",
  "term_label": "Unknown biological process",
  "gene_name": "Uroplakin-1b",
  "gene_symbol": "UPK1B"
}